{
  "gene_name": "Cell division cycle protein 23 homolog",
  "gene": "UniProtKB:Q9UJX2",
  "term_label": "protein ubiquitination",
  "term_id": "GO:0016567",
  "gene_symbol": "CDC23"
}